{
  "gene_name": "Ubiquitin carboxyl-terminal hydrolase 28",
  "gene": "UniProtKB:Q96RU2",
  "term_label": "regulation of protein stability",
  "term_id": "GO:0031647",
  "gene_symbol": "USP28"
}